{
  "term_id": "GO:0005634",
  "gene": "UniProtKB:Q9P0M6",
  "term_label": "nucleus",
  "gene_symbol": "MACROH2A2",
  "gene_name": "Core histone macro-H2A.2"
}